voltage-gated monoatomic anion channel activity [GO:0008308] (molecular function) Definition: Enables the transmembrane transfer of an anion by a voltage-gated channel. An anion is a negatively charged ion. A voltage-gated channel is a channel whose open state is dependent on the voltage across the membrane in which it is embedded. Relationships: is a type of GO:0005244; is a type of monoatomic anion channel activity [GO:0005253] Also known as: voltage-gated anion channel activity, voltage-dependent ion-selective channel activity, voltage-gated ion-selective channel activity Subtypes: GO:0005247 Sources: GOC:mtg_transport, GOC:vw, ISBN:0815340729